{
  "gene_name": "DENN domain-containing protein 1A",
  "gene": "UniProtKB:Q8TEH3",
  "term_id": "GO:1901981",
  "gene_symbol": "DENND1A",
  "term_label": "phosphatidylinositol phosphate binding"
}